{
  "term_id": "GO:0004197",
  "gene_symbol": "CASP8",
  "gene_name": "Caspase-8",
  "gene": "UniProtKB:Q14790",
  "term_label": "cysteine-type endopeptidase activity"
}